{
  "gene": "UniProtKB:Q96NW4",
  "gene_name": "Ankyrin repeat domain-containing protein 27",
  "term_id": "GO:0045022",
  "gene_symbol": "ANKRD27",
  "term_label": "early endosome to late endosome transport"
}